{
  "gene_symbol": "DERL2",
  "term_label": "endoplasmic reticulum unfolded protein response",
  "gene_name": "Derlin-2",
  "term_id": "GO:0030968",
  "gene": "UniProtKB:Q9GZP9"
}